{
  "gene_symbol": "CNTNAP5",
  "term_id": "UNKNOWN:0001",
  "gene_name": "Contactin-associated protein-like 5",
  "term_label": "Unknown molecular function",
  "gene": "UniProtKB:Q8WYK1"
}